{
  "gene": "UniProtKB:Q969E4",
  "gene_symbol": "TCEAL3",
  "gene_name": "Transcription elongation factor A protein-like 3",
  "term_id": "UNKNOWN:0001",
  "term_label": "Unknown molecular function"
}